{
  "term_id": "GO:0031125",
  "gene_name": "RNA exonuclease 5",
  "gene_symbol": "REXO5",
  "term_label": "rRNA 3'-end processing",
  "gene": "UniProtKB:Q96IC2"
}